chloroplast mRNA modification [GO:1900871] (biological process) References: PMID:1653905 Sources: GOC:TermGenie Relationships: is a type of mRNA modification [GO:0016556]; is a type of chloroplast RNA modification [GO:1900865] Also known as: chloroplast mRNA editing, mRNA editing in chloroplast Definition: The covalent alteration within the chloroplast of one or more nucleotides within an mRNA to produce an mRNA molecule with a sequence that differs from that coded genetically.